{
  "term_label": "Unknown molecular function",
  "gene": "UniProtKB:Q14166",
  "term_id": "UNKNOWN:0001",
  "gene_symbol": "TTLL12",
  "gene_name": "Tubulin--tyrosine ligase-like protein 12"
}